{
  "term_id": "GO:0048240",
  "gene": "UniProtKB:Q9NTU4",
  "gene_symbol": "CATSPERZ",
  "term_label": "sperm capacitation",
  "gene_name": "Cation channel sperm-associated auxiliary subunit zeta"
}